{
  "term_label": "protein kinase binding",
  "gene_name": "Protein FAM83A",
  "gene": "UniProtKB:Q86UY5",
  "gene_symbol": "FAM83A",
  "term_id": "GO:0019901"
}